{
  "gene_name": "Ras-related protein Rab-5A",
  "term_label": "plasma membrane",
  "gene": "UniProtKB:P20339",
  "gene_symbol": "RAB5A",
  "term_id": "GO:0005886"
}